{
  "term_id": "GO:0004843",
  "gene_name": "Ubiquitin carboxyl-terminal hydrolase 17-like protein 21",
  "gene_symbol": "USP17L21",
  "gene": "UniProtKB:D6R901",
  "term_label": "cysteine-type deubiquitinase activity"
}